{
  "term_id": "GO:0000165",
  "gene_symbol": "MAP2K5",
  "term_label": "MAPK cascade",
  "gene_name": "Dual specificity mitogen-activated protein kinase kinase 5",
  "gene": "UniProtKB:Q13163"
}